{
  "term_id": "UNKNOWN:0001",
  "gene_symbol": "DEFB105B",
  "term_label": "Unknown molecular function",
  "gene": "UniProtKB:Q8NG35",
  "gene_name": "Beta-defensin 105"
}